type I protein secretion system complex [GO:0030256] (CC) Definition: A complex of three secretory proteins that carry out secretion in the type I secretion system: an inner membrane transport ATPase (termed ABC protein for ATP-binding cassette), which provides the energy for protein secretion; an outer membrane protein, which is exported via the sec pathway; and a membrane fusion protein, which is anchored in the inner membrane and spans the periplasmic space. References: PMID:9618447 Also known as: ABC translocator complex Relationships: is a type of protein-containing complex [GO:0032991]